{
  "term_label": "Unknown biological process",
  "term_id": "UNKNOWN:0002",
  "gene_name": "Glomulin",
  "gene": "UniProtKB:Q92990",
  "gene_symbol": "GLMN"
}